{
  "term_label": "immunoglobulin complex",
  "gene_name": "Immunoglobulin kappa variable 3D-11",
  "gene": "UniProtKB:A0A0A0MRZ8",
  "gene_symbol": "IGKV3D-11",
  "term_id": "GO:0019814"
}